{
  "gene_symbol": "EN1",
  "gene_name": "Homeobox protein engrailed-1",
  "term_id": "GO:0006357",
  "term_label": "regulation of transcription by RNA polymerase II",
  "gene": "UniProtKB:Q05925"
}